{
  "term_label": "positive regulation of transcription by RNA polymerase II",
  "term_id": "GO:0045944",
  "gene": "UniProtKB:Q14541",
  "gene_name": "Hepatocyte nuclear factor 4-gamma",
  "gene_symbol": "HNF4G"
}